{
  "gene_symbol": "SLC24A5",
  "term_label": "trans-Golgi network",
  "gene": "UniProtKB:Q71RS6",
  "term_id": "GO:0005802",
  "gene_name": "Sodium_potassium_calcium exchanger 5"
}